monosaccharide catabolic process [GO:0046365] (biological process) Sources: ISBN:0198506732 Also known as: monosaccharide breakdown, monosaccharide catabolism, monosaccharide degradation Definition: The chemical reactions and pathways resulting in the breakdown of monosaccharides, polyhydric alcohols containing either an aldehyde or a keto group and between three to ten or more carbon atoms. Subtypes: GO:0019320, pentose catabolic process [GO:0019323], D-galacturonate catabolic process [GO:0019698], GO:0019854, 2-dehydro-3-deoxy-D-gluconic acid catabolic process [GO:1901273], 1,5-anhydro-D-fructose catabolic process [GO:1901802] Relationships: is a type of GO:0005996; is a type of carbohydrate catabolic process [GO:0016052]; is a type of small molecule catabolic process [GO:0044282]